{
  "term_id": "GO:0004711",
  "gene": "UniProtKB:Q9UK32",
  "gene_name": "Ribosomal protein S6 kinase alpha-6",
  "gene_symbol": "RPS6KA6",
  "term_label": "ribosomal protein S6 kinase activity"
}